{
  "gene": "UniProtKB:Q5VTH2",
  "term_id": "GO:0036064",
  "gene_symbol": "CFAP126",
  "gene_name": "Protein Flattop",
  "term_label": "ciliary basal body"
}